L-amino acid catabolic process [GO:0170035] (biological process) Definition: The chemical reactions and pathways resulting in the breakdown of an L-amino acid. Also known as: L-amino acid breakdown, L-amino acid catabolism, L-amino acid degradation Sources: GOC:edw Relationships: is a type of L-amino acid metabolic process [GO:0170033]; is a type of GO:1901606 Subtypes: L-arginine catabolic process [GO:0006527], L-asparagine catabolic process [GO:0006530], GO:0006533, L-glutamate catabolic process [GO:0006538], GO:0006543, L-histidine catabolic process [GO:0006548], L-isoleucine catabolic process [GO:0006550], L-leucine catabolic process [GO:0006552], L-phenylalanine catabolic process [GO:0006559], GO:0006562, L-serine catabolic process [GO:0006565], GO:0006567, GO:0006569, L-tyrosine catabolic process [GO:0006572], L-valine catabolic process [GO:0006574], L-ornithine catabolic process [GO:0006593], L-methionine catabolic process [GO:0009087], GO:0019448, GO:0019470, L-lysine catabolic process [GO:0019477], L-proline betaine catabolic process [GO:0019504], S-adenosylhomocysteine catabolic process [GO:0019510], discadenine catabolic process [GO:0034269], L-alanine catabolic process [GO:0042853], phosphoarginine catabolic process [GO:0046313], L-kynurenine catabolic process [GO:0097053], 3-cyano-L-alanine catabolic process [GO:1903559], GO:2001297, N(omega),N(omega)-dimethyl-L-arginine catabolic process [GO:2001299]